{
  "gene_name": "Growth factor receptor-bound protein 7",
  "gene": "UniProtKB:Q14451",
  "term_label": "Unknown cellular component",
  "term_id": "UNKNOWN:0003",
  "gene_symbol": "GRB7"
}